NADP+ nucleosidase activity [GO:0050135] (molecular function) Sources: RHEA:19849 Also known as: NAD(P)+ nucleosidase activity, NADP nucleosidase activity, NADP(+) nucleosidase activity, NADP+ glycohydrolase activity, NADPase activity Definition: Catalysis of the reaction: NADP+ + H2O = ADP-D-ribose 2'-phosphate + nicotinamide + H+. Relationships: is a type of hydrolase activity, hydrolyzing N-glycosyl compounds [GO:0016799]